{
  "gene_name": "PHD finger protein 20",
  "gene_symbol": "PHF20",
  "gene": "UniProtKB:Q9BVI0",
  "term_label": "MLL1 complex",
  "term_id": "GO:0071339"
}